{
  "gene": "UniProtKB:Q9NP79",
  "term_label": "multivesicular body",
  "term_id": "GO:0005771",
  "gene_name": "Vacuolar protein sorting-associated protein VTA1 homolog",
  "gene_symbol": "VTA1"
}